{
  "gene_name": "PRAME family member 12",
  "gene": "UniProtKB:O95522",
  "term_id": "GO:0043161",
  "term_label": "proteasome-mediated ubiquitin-dependent protein catabolic process",
  "gene_symbol": "PRAMEF12"
}